{
  "gene": "UniProtKB:Q9NVV9",
  "gene_name": "THAP domain-containing protein 1",
  "term_id": "GO:0000978",
  "gene_symbol": "THAP1",
  "term_label": "RNA polymerase II cis-regulatory region sequence-specific DNA binding"
}